{
  "gene": "UniProtKB:Q9UHE5",
  "term_id": "UNKNOWN:0003",
  "gene_symbol": "NAT8",
  "term_label": "Unknown cellular component",
  "gene_name": "N-acetyltransferase 8"
}